metanephric connecting tubule development [GO:0072286] (biological process) Definition: The process whose specific outcome is the progression of the metanephric connecting tubule over time, from its formation to the mature structure. The metanephric connecting tubule is a tubular segment of the metanephric nephron; it connects the distal convoluted tubule to the collecting duct in the metanephros. Relationships: is a type of GO:0072027; is_a metanephric nephron tubule development [GO:0072234] Sources: GOC:mtg_kidney_jan10 Also known as: metanephric connecting duct development